{
  "gene_name": "Zinc finger protein 407",
  "term_id": "GO:0006355",
  "gene": "UniProtKB:Q9C0G0",
  "term_label": "regulation of DNA-templated transcription",
  "gene_symbol": "ZNF407"
}